{
  "term_label": "protein folding",
  "gene_name": "DnaJ homolog subfamily B member 13",
  "gene": "UniProtKB:P59910",
  "term_id": "GO:0006457",
  "gene_symbol": "DNAJB13"
}